membrane repolarization during atrial cardiac muscle cell action potential [GO:0098914] (biological process) Also known as: atrial repolarization, electrocardiogram QRS complex Regulation: regulated by regulation of membrane repolarization during atrial cardiac muscle cell action potential [GO:1905000]; negatively regulated by negative regulation of membrane repolarization during atrial cardiac muscle cell action potential [GO:1905001]; positively regulated by positive regulation of membrane repolarization during atrial cardiac muscle cell action potential [GO:1905002] Sources: GOC:dph, GOC:mtg_cardiac_conduct_nov11, GOC:tb Definition: The process in which ions are transported across a membrane such that the atrial cardiomyocyte membrane potential changes in the direction from the positive membrane potential at the peak of the action potential towards the negative resting potential. Relationships: is a type of membrane repolarization during cardiac muscle cell action potential [GO:0086013]; is a type of atrial cardiac muscle cell membrane repolarization [GO:0099624]; is part of atrial cardiac muscle cell action potential [GO:0086014]